neuromedin U binding [GO:0042924] (molecular function) Definition: Interacting selectively and non-covalently and stoichiometrically with neuromedin U, a hypothalamic peptide involved in energy homeostasis and stress responses. Relationships: is a type of neuropeptide binding [GO:0042923] References: PMID:12584108 Sources: GOC:jl Also known as: NMU binding